negative regulation of catalytic activity [GO:0043086] (biological process) Relationships: is a type of GO:0044092; is a type of regulation of catalytic activity [GO:0050790]; negatively regulates catalytic activity [GO:0003824] Subtypes: negative regulation of adenylate cyclase activity [GO:0007194], negative regulation of protein ADP-ribosylation [GO:0010836], negative regulation of guanylate cyclase activity [GO:0031283], negative regulation of kinase activity [GO:0033673], negative regulation of helicase activity [GO:0051097], GO:0051346, negative regulation of oxidoreductase activity [GO:0051354], negative regulation of ubiquitin-protein transferase activity [GO:0051444], negative regulation of endoribonuclease activity [GO:0060702], negative regulation of RNA-dependent RNA polymerase activity [GO:1900260], negative regulation of polynucleotide adenylyltransferase activity [GO:1904246], GO:2000466 Also known as: down regulation of enzyme activity, down-regulation of enzyme activity, down-regulation of metalloenzyme activity, downregulation of enzyme activity, negative regulation of enzyme activity, down regulation of metalloenzyme activity, downregulation of metalloenzyme activity, inhibition of enzyme activity, inhibition of metalloenzyme activity, negative regulation of metalloenzyme activity Definition: Any process that stops or reduces the activity of an enzyme. Sources: GOC:ebc, GOC:jl, GOC:tb, GOC:vw